{
  "gene": "UniProtKB:Q9NVG8",
  "gene_name": "TBC1 domain family member 13",
  "gene_symbol": "TBC1D13",
  "term_id": "GO:0005096",
  "term_label": "GTPase activator activity"
}